ureter part of ureteric bud development [GO:0035503] (biological process) Definition: The development of the portion of the ureteric bud that contributes to the morphogenesis of the ureter. The ureter ureteric bud is the initial structure that forms the ureter. Sources: GOC:mtg_kidney_jan10 Relationships: is a type of tube development [GO:0035295]; is part of ureteric bud development [GO:0001657]; is part of ureter morphogenesis [GO:0072197]